{
  "gene_name": "YTH domain-containing family protein 3",
  "gene": "UniProtKB:Q7Z739",
  "gene_symbol": "YTHDF3",
  "term_id": "GO:0061157",
  "term_label": "mRNA destabilization"
}